{
  "gene_symbol": "SPAG11B",
  "gene": "UniProtKB:Q08648",
  "term_id": "UNKNOWN:0002",
  "term_label": "Unknown biological process",
  "gene_name": "Sperm-associated antigen 11B"
}